apical tubulobulbar complex [GO:0061828] (cellular component) Also known as: apical TBC References: PMID:20403871, PMID:22510523 Definition: Actin-based structures involved in establishing close contact between mature spermatids and Sertoli cells at the luminal end of the Sertoli cell. Relationships: is a type of tubulobulbar complex [GO:0036284]